{
  "gene": "UniProtKB:Q9BRJ9",
  "gene_symbol": "MESP1",
  "term_id": "GO:0005634",
  "gene_name": "Mesoderm posterior protein 1",
  "term_label": "nucleus"
}